{
  "term_id": "GO:0005789",
  "gene_name": "Long-chain fatty acid transport protein 6",
  "gene": "UniProtKB:Q9Y2P4",
  "gene_symbol": "SLC27A6",
  "term_label": "endoplasmic reticulum membrane"
}